sorbose 5-dehydrogenase (NADP+) activity [GO:0050287] (molecular function) Also known as: 5-keto-D-fructose reductase activity, 5-ketofructose reductase activity, L-sorbose:NADP+ 5-oxidoreductase activity, reduced nicotinamide adenine dinucleotide phosphate-linked reductase activity, sorbose (nicotinamide adenine dinucleotide phosphate) dehydrogenase activity Relationships: is a type of oxidoreductase activity, acting on the CH-OH group of donors, NAD or NADP as acceptor [GO:0016616] Sources: EC:1.1.1.123, RHEA:15001 Definition: Catalysis of the reaction: L-sorbose + NADP+ = 5-dehydro-D-fructose + H+ + NADPH.